{
  "gene": "UniProtKB:O43306",
  "gene_name": "Adenylate cyclase type 6",
  "term_id": "GO:0006171",
  "term_label": "cAMP biosynthetic process",
  "gene_symbol": "ADCY6"
}